{
  "gene_symbol": "ARHGAP39",
  "term_id": "GO:0005096",
  "gene_name": "Rho GTPase-activating protein 39",
  "gene": "UniProtKB:Q9C0H5",
  "term_label": "GTPase activator activity"
}